{
  "term_id": "GO:0000086",
  "gene_name": "Cyclin-dependent kinase 3",
  "gene": "UniProtKB:Q00526",
  "term_label": "G2/M transition of mitotic cell cycle",
  "gene_symbol": "CDK3"
}